{
  "gene_symbol": "CCDC17",
  "gene": "UniProtKB:Q96LX7",
  "gene_name": "Coiled-coil domain-containing protein 17",
  "term_id": "UNKNOWN:0002",
  "term_label": "Unknown biological process"
}